{
  "term_id": "GO:0005737",
  "gene_name": "G-protein coupled receptor 3",
  "term_label": "cytoplasm",
  "gene": "UniProtKB:P46089",
  "gene_symbol": "GPR3"
}